{
  "term_label": "actin cytoskeleton organization",
  "gene": "UniProtKB:Q76I76",
  "term_id": "GO:0030036",
  "gene_name": "Protein phosphatase Slingshot homolog 2",
  "gene_symbol": "SSH2"
}